{
  "gene": "UniProtKB:P0DI81",
  "term_id": "GO:0005634",
  "gene_name": "Trafficking protein particle complex subunit 2",
  "term_label": "nucleus",
  "gene_symbol": "TRAPPC2"
}